{
  "term_label": "maturation of SSU-rRNA from tricistronic rRNA transcript (SSU-rRNA, 5.8S rRNA, LSU-rRNA)",
  "gene_name": "WD repeat-containing protein 46",
  "gene_symbol": "WDR46",
  "gene": "UniProtKB:O15213",
  "term_id": "GO:0000462"
}